regulation of bile acid secretion [GO:0120188] (BP) Relationships: is a type of GO:0032890; is a type of GO:0051046; regulates bile acid secretion [GO:0032782] References: PMID:22767443 Sources: GOC:BHF, GOC:BHF_miRNA, GOC:rph Subtypes: positive regulation of bile acid secretion [GO:0120189], negative regulation of bile acid secretion [GO:0120190] Definition: Any process that modulates the frequency, rate or extent of the controlled release of bile acid from a cell or a tissue.